cytosine transmembrane transporter activity [GO:0015209] (molecular function) Relationships: is a type of pyrimidine nucleobase transmembrane transporter activity [GO:0005350]; is part of GO:0015856 Sources: GOC:go_curators Subtypes: cytosine:proton symporter activity [GO:0015504] Definition: Enables the transfer of cytosine, 4-amino-2-hydroxypyrimidine from one side of a membrane to the other.